{
  "gene_symbol": "DCTN5",
  "term_label": "Unknown molecular function",
  "gene": "UniProtKB:Q9BTE1",
  "gene_name": "Dynactin subunit 5",
  "term_id": "UNKNOWN:0001"
}